homospermidine synthase activity [GO:0047296] (molecular function) Definition: Catalysis of the reaction: 2 putrescine = NH3 + sym-homospermidine. Relationships: is a type of GO:0016765 Sources: EC:2.5.1.44, MetaCyc:2.5.1.44-RXN Also known as: putrescine:putrescine 4-aminobutyltransferase (ammonia-forming)